{
  "gene": "UniProtKB:Q9HBH7",
  "gene_symbol": "BEX1",
  "gene_name": "Protein BEX1",
  "term_label": "nucleus",
  "term_id": "GO:0005634"
}